{
  "term_id": "GO:0000177",
  "gene": "UniProtKB:Q13868",
  "gene_name": "Exosome complex component RRP4",
  "gene_symbol": "EXOSC2",
  "term_label": "cytoplasmic exosome (RNase complex)"
}